acetaldehyde catabolic process [GO:0046187] (biological process) Relationships: is_a acetaldehyde metabolic process [GO:0006117]; is a type of GO:0046185 Also known as: acetaldehyde breakdown, acetaldehyde catabolism, acetaldehyde degradation Sources: GOC:ai Definition: The chemical reactions and pathways resulting in the breakdown of acetaldehyde, a colorless, flammable liquid intermediate in the metabolism of alcohol.